{
  "gene_name": "Catenin alpha-1",
  "term_id": "GO:0016477",
  "gene": "UniProtKB:P35221",
  "term_label": "cell migration",
  "gene_symbol": "CTNNA1"
}